petal development [GO:0048441] (biological process) Relationships: is_a floral organ development [GO:0048437]; is_a GO:0048827; is part of GO:0048465 Sources: GOC:go_curators Definition: The process whose specific outcome is the progression of the petal over time, from its formation to the mature structure.